{
  "term_id": "GO:0007411",
  "gene_name": "Semaphorin-4A",
  "gene": "UniProtKB:Q9H3S1",
  "gene_symbol": "SEMA4A",
  "term_label": "axon guidance"
}